gibberellin binding [GO:0010331] (molecular function) Relationships: is a type of isoprenoid binding [GO:0019840]; is_a GO:0031406; is a type of GO:0042562 Also known as: gibberellic acid receptor, gibberellin receptor Definition: Binding to a gibberellin, a plant hormone that regulates aspects of plant growth. Sources: GOC:tair_curators